{
  "term_label": "Unknown cellular component",
  "term_id": "UNKNOWN:0003",
  "gene_symbol": "ERVK-25",
  "gene": "UniProtKB:P63136",
  "gene_name": "Endogenous retrovirus group K member 25 Pol protein"
}